{
  "gene_symbol": "JPT1",
  "term_label": "Unknown molecular function",
  "term_id": "UNKNOWN:0001",
  "gene_name": "Jupiter microtubule associated homolog 1",
  "gene": "UniProtKB:Q9UK76"
}